dendritic spine morphogenesis [GO:0060997] (biological process) Definition: The process in which the anatomical structures of a dendritic spine are generated and organized. A dendritic spine is a protrusion from a dendrite and a specialized subcellular compartment involved in synaptic transmission. Sources: GOC:dph Relationships: is_a neuron projection development [GO:0031175]; is a type of neuron projection morphogenesis [GO:0048812]; is a type of GO:0097061; is part of dendrite morphogenesis [GO:0048813]; is part of dendritic spine development [GO:0060996] Regulation: regulated by regulation of dendritic spine morphogenesis [GO:0061001]; negatively regulated by negative regulation of dendritic spine morphogenesis [GO:0061002]; positively regulated by positive regulation of dendritic spine morphogenesis [GO:0061003]